{
  "gene_symbol": "A0A0G2JQF1",
  "gene": "UniProtKB:A0A0G2JQF1",
  "gene_name": "Uncharacterized protein",
  "term_label": "Unknown cellular component",
  "term_id": "UNKNOWN:0003"
}